regulation of systemic arterial blood pressure by norepinephrine [GO:0003048] (biological process) Relationships: is a type of regulation of systemic arterial blood pressure mediated by a chemical signal [GO:0003044]; is part of GO:0001993 Also known as: regulation of blood pressure by noradrenaline, blood pressure regulation by norepinephrine Sources: GOC:mtg_cardio Definition: The regulation of blood pressure mediated by the catecholamine signaling molecule norepinephrine.